{
  "gene_name": "Cell cycle checkpoint protein RAD1",
  "term_label": "DNA repair",
  "gene": "UniProtKB:O60671",
  "term_id": "GO:0006281",
  "gene_symbol": "RAD1"
}